meiotic cell cycle process involved in oocyte maturation [GO:1903537] (biological process) Regulation: regulated by GO:1903538; negatively regulated by negative regulation of meiotic cell cycle process involved in oocyte maturation [GO:1904145]; positively regulated by positive regulation of meiotic cell cycle process involved in oocyte maturation [GO:1904146] Definition: Any meiotic cell cycle process that is involved in oocyte maturation. Also known as: meiosis involved in oocyte maturation References: PMID:25212395 Sources: GOC:TermGenie, GOC:jz, GO_REF:0000060 Relationships: is a type of GO:1903046; is part of oocyte maturation [GO:0001556]